{
  "term_id": "GO:0036128",
  "gene_name": "Cation channel sperm-associated protein 4",
  "term_label": "CatSper complex",
  "gene_symbol": "CATSPER4",
  "gene": "UniProtKB:Q7RTX7"
}